pancreatic D cell development [GO:0003324] (biological process) Definition: The process whose specific outcome is the progression of a pancreatic delta cell over time, from its formation to the mature structure. A delta cell is a cell of the pancreas that produces somatostatin. Relationships: is a type of columnar/cuboidal epithelial cell development [GO:0002066]; is a type of neuron development [GO:0048666]; BFO_0000050 pancreatic D cell differentiation [GO:0003311] Sources: GOC:dph Also known as: pancreatic delta cell development